{
  "term_id": "GO:0046856",
  "term_label": "phosphatidylinositol dephosphorylation",
  "gene_symbol": "MTMR7",
  "gene_name": "Myotubularin-related protein 7",
  "gene": "UniProtKB:Q9Y216"
}